negative regulation of Wnt-Frizzled-LRP5/6 complex assembly [GO:1904723] (biological process) References: PMID:11433302 Sources: GOC:PARL, GOC:TermGenie, GOC:bf, GO_REF:0000058 Relationships: is_a GO:0031333; is a type of regulation of Wnt-Frizzled-LRP5/6 complex assembly [GO:1904711]; negatively regulates Wnt-Frizzled-LRP5/6 complex assembly [GO:1904701] Also known as: down regulation of Frizzled-LRP5/6 complex assembly, down regulation of Wnt-FZD-LRP5/6 trimeric complex assembly, down regulation of Wnt-FZD-LRP5/6 trimeric complex formation, down-regulation of Frizzled-LRP5/6 complex assembly, down-regulation of Wnt-FZD-LRP5/6 trimeric complex assembly, down-regulation of Wnt-FZD-LRP5/6 trimeric complex formation, downregulation of Frizzled-LRP5/6 complex assembly, downregulation of Wnt-FZD-LRP5/6 trimeric complex assembly, downregulation of Wnt-FZD-LRP5/6 trimeric complex formation, negative regulation of Wnt-FZD-LRP5/6 trimeric complex assembly, negative regulation of Wnt-FZD-LRP5/6 trimeric complex formation, down regulation of WNT-FZD-LRP5 complex assembly, down regulation of WNT-FZD-LRP5 complex formation, down regulation of WNT-FZD-LRP6 complex assembly, down regulation of WNT-FZD-LRP6 complex formation, down-regulation of WNT-FZD-LRP5 complex assembly, down-regulation of WNT-FZD-LRP5 complex formation, down-regulation of WNT-FZD-LRP6 complex assembly, down-regulation of WNT-FZD-LRP6 complex formation, downregulation of WNT-FZD-LRP5 complex assembly, downregulation of WNT-FZD-LRP5 complex formation, downregulation of WNT-FZD-LRP6 complex assembly, downregulation of WNT-FZD-LRP6 complex formation, inhibition of Frizzled-LRP5/6 complex assembly, inhibition of WNT-FZD-LRP5 complex assembly, inhibition of WNT-FZD-LRP5 complex formation, inhibition of WNT-FZD-LRP6 complex assembly, inhibition of WNT-FZD-LRP6 complex formation, inhibition of Wnt-FZD-LRP5/6 trimeric complex assembly, inhibition of Wnt-FZD-LRP5/6 trimeric complex formation, negative regulation of WNT-FZD-LRP5 complex assembly, negative regulation of WNT-FZD-LRP5 complex formation, negative regulation of WNT-FZD-LRP6 complex assembly, negative regulation of WNT-FZD-LRP6 complex formation, down regulation of Frizzled-LRP5/6 complex formation, down regulation of Wnt-induced Frizzled-LRP5/6 complex assembly, down regulation of Wnt-induced Frizzled-LRP5/6 complex formation, down-regulation of Frizzled-LRP5/6 complex formation, down-regulation of Wnt-induced Frizzled-LRP5/6 complex assembly, down-regulation of Wnt-induced Frizzled-LRP5/6 complex formation, downregulation of Frizzled-LRP5/6 complex formation, downregulation of Wnt-induced Frizzled-LRP5/6 complex assembly, downregulation of Wnt-induced Frizzled-LRP5/6 complex formation, inhibition of Frizzled-LRP5/6 complex formation, inhibition of Wnt-induced Frizzled-LRP5/6 complex assembly, inhibition of Wnt-induced Frizzled-LRP5/6 complex formation, negative regulation of Frizzled-LRP5/6 complex assembly, negative regulation of Frizzled-LRP5/6 complex formation, negative regulation of Wnt-induced Frizzled-LRP5/6 complex assembly, negative regulation of Wnt-induced Frizzled-LRP5/6 complex formation Definition: Any process that stops, prevents or reduces the frequency, rate or extent of Wnt-Frizzled-LRP5/6 complex assembly.